{
  "gene": "UniProtKB:P21917",
  "gene_name": "D(4) dopamine receptor",
  "term_label": "G protein-coupled serotonin receptor activity",
  "gene_symbol": "DRD4",
  "term_id": "GO:0004993"
}